tRNA splicing, via endonucleolytic cleavage and ligation [GO:0006388] (BP) Also known as: tRNA-Y splicing Note: Note that while typically associated with tRNA splicing, splicing via endonucleolytic cleavages and subsequent ligation of the free exon ends is known to be used for some non-tRNA substrates, e.g. HAC1 (YFL031W) in S. cerevisiae and an intron in the 23S rRNA of the Archaeal species Desulfurococcus mobilis. Relationships: is a type of RNA splicing, via endonucleolytic cleavage and ligation [GO:0000394]; is a type of tRNA processing [GO:0008033] Definition: Splicing of tRNA substrates via recognition of the folded RNA structure that brings the 5' and 3' splice sites into proximity and cleavage of the RNA at both the 3' and 5' splice sites by an endonucleolytic mechanism, followed by ligation of the exons. References: PMID:9582290 Sources: GOC:krc, ISBN:0879695897